{
  "term_label": "Unknown molecular function",
  "gene_symbol": "ARHGEF35",
  "gene_name": "Rho guanine nucleotide exchange factor 35",
  "term_id": "UNKNOWN:0001",
  "gene": "UniProtKB:A5YM69"
}